{
  "term_label": "Unknown molecular function",
  "term_id": "UNKNOWN:0001",
  "gene": "UniProtKB:Q5TIE3",
  "gene_symbol": "VWA5B1",
  "gene_name": "von Willebrand factor A domain-containing protein 5B1"
}